{
  "term_id": "GO:0006346",
  "gene_symbol": "MBD3",
  "term_label": "DNA methylation-dependent constitutive heterochromatin formation",
  "gene_name": "Methyl-CpG-binding domain protein 3",
  "gene": "UniProtKB:O95983"
}